{
  "gene_name": "Transmembrane channel-like protein 7",
  "term_label": "mechanosensitive monoatomic ion channel activity",
  "gene_symbol": "TMC7",
  "gene": "UniProtKB:Q7Z402",
  "term_id": "GO:0008381"
}